structural constituent of skin epidermis [GO:0030280] (molecular function) Definition: The action of a molecule that contributes to the structural integrity of an epidermal cutaneous structure. Also known as: structural constituent of epidermis Relationships: is a type of structural molecule activity [GO:0005198] Sources: GOC:mah